ceramide 1-phosphate transport [GO:1902389] (biological process) Relationships: is_a organic anion transport [GO:0015711]; is a type of phospholipid transport [GO:0015914]; is a type of GO:0035627 References: PMID:23863933 Sources: GOC:TermGenie Definition: The directed movement of a ceramide 1-phosphate into, out of or within a cell, or between cells, by means of some agent such as a transporter or pore.